symbiont-mediated pore formation in host plasma membrane [GO:0044658] (biological process) References: PMID:7510043 Sources: GOC:jl Definition: The disruption of host plasma membrane integrity by formation of a pore, resulting in deregulated ion homeostasis, and cellular dysfunction that can result in cell death. Also known as: pore formation in membrane of host by symbiont, pore formation in host plasma membrane Relationships: is a type of symbiont-mediated perturbation of host membrane [GO:0141171]